beta-glucan transmembrane transporter activity [GO:0015160] (molecular function) Definition: Enables the transfer of beta-glucans from one side of a membrane to the other. Beta-glucans are compounds composed of glucose residues linked by beta-glucosidic bonds. Subtypes: ABC-type beta-glucan transporter activity [GO:0015441] Sources: GOC:ai, GOC:mtg_transport, ISBN:0815340729 Relationships: is a type of polysaccharide transmembrane transporter activity [GO:0015159]; is part of beta-glucan transport [GO:0015775]